brain development [GO:0007420] (biological process) Relationships: is a type of animal organ development [GO:0048513]; is part of central nervous system development [GO:0007417]; is part of head development [GO:0060322] Sources: GOC:dph, GOC:jid, GOC:tb, UBERON:0000955 Definition: The process whose specific outcome is the progression of the brain over time, from its formation to the mature structure. Brain development begins with patterning events in the neural tube and ends with the mature structure that is the center of thought and emotion. The brain is responsible for the coordination and control of bodily activities and the interpretation of information from the senses (sight, hearing, smell, etc.).